{
  "gene": "UniProtKB:O15554",
  "gene_symbol": "KCNN4",
  "term_id": "GO:0005886",
  "gene_name": "Intermediate conductance calcium-activated potassium channel protein 4",
  "term_label": "plasma membrane"
}